{
  "term_label": "Unknown cellular component",
  "gene_symbol": "CLIC6",
  "term_id": "UNKNOWN:0003",
  "gene_name": "Chloride intracellular channel protein 6",
  "gene": "UniProtKB:Q96NY7"
}